{
  "term_label": "Unknown cellular component",
  "term_id": "UNKNOWN:0003",
  "gene_symbol": "TENT2",
  "gene": "UniProtKB:Q6PIY7",
  "gene_name": "Poly(A) RNA polymerase GLD2"
}